{
  "gene_name": "Folate receptor gamma",
  "term_id": "GO:0035036",
  "gene_symbol": "FOLR3",
  "gene": "UniProtKB:P41439",
  "term_label": "sperm-egg recognition"
}